{
  "gene_symbol": "SLC6A15",
  "gene_name": "Sodium-dependent neutral amino acid transporter B(0)AT2",
  "gene": "UniProtKB:Q9H2J7",
  "term_id": "GO:0035725",
  "term_label": "sodium ion transmembrane transport"
}